negative regulation of filamentous growth of a population of unicellular organisms in response to neutral pH [GO:1900441] (biological process) Relationships: is a type of regulation of filamentous growth of a population of unicellular organisms in response to neutral pH [GO:1900440]; is a type of negative regulation of filamentous growth of a population of unicellular organisms in response to pH [GO:1900742]; negatively regulates filamentous growth of a population of unicellular organisms in response to neutral pH [GO:0036178] Definition: Any process that stops, prevents or reduces the frequency, rate or extent of filamentous growth of a population of unicellular organisms in response to neutral pH. Sources: GOC:TermGenie, GOC:di Also known as: down regulation of filamentous growth of a population of unicellular organisms in response to neutral pH, down-regulation of filamentous growth of a population of unicellular organisms in response to neutral pH, downregulation of filamentous growth of a population of unicellular organisms in response to neutral pH, inhibition of filamentous growth of a population of unicellular organisms in response to neutral pH